{
  "gene_name": "Taste receptor type 2 member 3",
  "gene_symbol": "TAS2R3",
  "term_id": "GO:0001580",
  "gene": "UniProtKB:Q9NYW6",
  "term_label": "detection of chemical stimulus involved in sensory perception of bitter taste"
}